{
  "gene": "UniProtKB:O60522",
  "term_label": "P granule organization",
  "gene_symbol": "TDRD6",
  "gene_name": "Tudor domain-containing protein 6",
  "term_id": "GO:0030719"
}